detection of increased carbon dioxide by aortic body chemoreceptor signaling [GO:0003034] (biological process) Definition: The process in which information about the levels of carbon dioxide are received and are converted to a molecular signal by chemoreceptors in an aortic body. Sources: GOC:mtg_cardio Also known as: detection of increased carbon dioxide by aortic body chemoreceptor signalling Relationships: is a type of GO:0003021; is part of detection of hypoxic conditions in blood by aortic body chemoreceptor signaling [GO:0003033]